{
  "gene_symbol": "XAF1",
  "term_label": "Unknown biological process",
  "gene_name": "XIAP-associated factor 1",
  "gene": "UniProtKB:Q6GPH4",
  "term_id": "UNKNOWN:0002"
}